{
  "gene": "UniProtKB:P35240",
  "term_id": "GO:0005178",
  "gene_name": "Merlin",
  "gene_symbol": "NF2",
  "term_label": "integrin binding"
}